cytosolic [4Fe-4S] assembly targeting complex [GO:0097361] (cellular component) References: PMID:23585563, PMID:23891004, PMID:34660592 Definition: A protein complex capable of condensing two 2Fe-2S clusters into one 4Fe-4S center in the cytoplasm and nucleus. In humans it consists of MMS19, CIAO1, CIAO2A/CIAO2B, CIAO3. MMS19, CIAO1 and CIAO2A/CIAO2B form a tight 'core' complex, whereas CIAO3 is an 'external' component of this complex. Relationships: is a type of intracellular protein-containing complex [GO:0140535]; is a type of iron-sulfur cluster assembly complex [GO:1990229] Also known as: CIA complex, CIA targeting complex, cytosolic iron-sulfur protein assembly complex